{
  "term_id": "GO:0019005",
  "gene": "UniProtKB:Q5XUX0",
  "term_label": "SCF ubiquitin ligase complex",
  "gene_symbol": "FBXO31",
  "gene_name": "F-box only protein 31"
}